{
  "term_id": "UNKNOWN:0003",
  "gene_name": "Vitamin K epoxide reductase complex subunit 1-like protein 1",
  "gene": "UniProtKB:Q8N0U8",
  "gene_symbol": "VKORC1L1",
  "term_label": "Unknown cellular component"
}